gap junction assembly [GO:0016264] (biological process) Sources: GOC:jid, ISBN:0716731363 Regulation: regulated by regulation of gap junction assembly [GO:1903596]; negatively regulated by negative regulation of gap junction assembly [GO:1903597]; positively regulated by positive regulation of gap junction assembly [GO:1903598] Definition: Assembly of gap junctions, which are found in most animal tissues, and serve as direct connections between the cytoplasms of adjacent cells. They provide open channels through the plasma membrane, allowing ions and small molecules (less than approximately a thousand daltons) to diffuse freely between neighboring cells, but preventing the passage of proteins and nucleic acids. Relationships: is a type of cell-cell junction assembly [GO:0007043]